{
  "gene": "UniProtKB:Q6K0P9",
  "gene_name": "Pyrin and HIN domain-containing protein 1",
  "term_label": "nucleoplasm",
  "term_id": "GO:0005654",
  "gene_symbol": "PYHIN1"
}